{
  "gene_symbol": "SYP",
  "gene_name": "Synaptophysin",
  "term_label": "presynaptic active zone",
  "term_id": "GO:0048786",
  "gene": "UniProtKB:P08247"
}